granulosa cell differentiation [GO:0060014] (biological process) Relationships: is a type of epithelial cell differentiation [GO:0030855] Definition: The process in which a relatively unspecialized cell acquires the specialized features of a granulosa cell, a supporting cell for the developing female gamete in the ovary of mammals. Sources: GOC:dph Subtypes: GO:0001549